{
  "term_id": "UNKNOWN:0001",
  "gene_name": "Meiosis expressed gene 1 protein homolog",
  "gene_symbol": "MEIG1",
  "term_label": "Unknown molecular function",
  "gene": "UniProtKB:Q5JSS6"
}